{
  "term_label": "sarcolemma",
  "gene_name": "Popeye domain-containing protein 2",
  "term_id": "GO:0042383",
  "gene_symbol": "POPDC2",
  "gene": "UniProtKB:Q9HBU9"
}